{
  "gene_symbol": "SYCP2",
  "gene": "UniProtKB:Q9BX26",
  "term_label": "Unknown biological process",
  "gene_name": "Synaptonemal complex protein 2",
  "term_id": "UNKNOWN:0002"
}